establishment of protein localization to vacuole [GO:0072666] (biological process) Sources: GOC:mah Relationships: is a type of establishment of protein localization to organelle [GO:0072594] Also known as: establishment of protein localisation to vacuole Definition: The directed movement of a protein to a specific location in a vacuole. Subtypes: protein targeting to vacuole [GO:0006623], protein transport to vacuole involved in ubiquitin-dependent protein catabolic process via the multivesicular body sorting pathway [GO:0043328], neurotransmitter receptor transport, postsynaptic endosome to lysosome [GO:0098943]